{
  "term_label": "renal system process",
  "term_id": "GO:0003014",
  "gene_symbol": "SLC4A5",
  "gene": "UniProtKB:Q9BY07",
  "gene_name": "Electrogenic sodium bicarbonate cotransporter 4"
}